{
  "term_label": "sphingolipid biosynthetic process",
  "gene": "UniProtKB:Q9NXB9",
  "gene_symbol": "ELOVL2",
  "term_id": "GO:0030148",
  "gene_name": "Elongation of very long chain fatty acids protein 2"
}